{
  "gene_symbol": "HBEGF",
  "gene": "UniProtKB:Q99075",
  "term_label": "epidermal growth factor receptor signaling pathway",
  "term_id": "GO:0007173",
  "gene_name": "Proheparin-binding EGF-like growth factor"
}